{
  "term_label": "muscle contraction",
  "gene_name": "Tropomyosin alpha-4 chain",
  "term_id": "GO:0006936",
  "gene": "UniProtKB:P67936",
  "gene_symbol": "TPM4"
}